{
  "gene_symbol": "CIAO2A",
  "gene": "UniProtKB:Q9H5X1",
  "term_id": "GO:0051604",
  "gene_name": "Cytosolic iron-sulfur assembly component 2A",
  "term_label": "protein maturation"
}